regulation of dehydroepiandrosterone secretion [GO:2000840] (biological process) Relationships: is a type of regulation of lipid transport [GO:0032368]; is a type of regulation of hormone secretion [GO:0046883]; regulates dehydroepiandrosterone secretion [GO:0035942] Also known as: regulation of 3beta-hydroxyandrost-5-en-17-one secretion, regulation of DHEA secretion, regulation of dehydroisoandrosterone secretion Definition: Any process that modulates the frequency, rate or extent of dehydroepiandrosterone secretion. Sources: GOC:sl Subtypes: negative regulation of dehydroepiandrosterone secretion [GO:2000841], positive regulation of dehydroepiandrosterone secretion [GO:2000842]